{
  "term_id": "UNKNOWN:0002",
  "gene_name": "T cell receptor gamma variable 5",
  "gene": "UniProtKB:A0A0B4J1U4",
  "gene_symbol": "TRGV5",
  "term_label": "Unknown biological process"
}